{
  "term_label": "N6-methyladenosine-containing RNA reader activity",
  "term_id": "GO:1990247",
  "gene_symbol": "YTHDC1",
  "gene_name": "YTH domain-containing protein 1",
  "gene": "UniProtKB:Q96MU7"
}